{
  "gene_symbol": "CRYBG3",
  "term_label": "visual perception",
  "gene": "UniProtKB:Q68DQ2",
  "gene_name": "Very large A-kinase anchor protein",
  "term_id": "GO:0007601"
}